protein kinase activator activity [GO:0030295] (molecular function) Relationships: is a type of GO:0019209; is_a protein kinase regulator activity [GO:0019887]; positively regulates protein kinase activity [GO:0004672] Sources: GOC:ai Subtypes: protein tyrosine kinase activator activity [GO:0030296], GO:0043539 Definition: Binds to and increases the activity of a protein kinase, an enzyme which phosphorylates a protein.